{
  "term_id": "GO:0033173",
  "gene": "UniProtKB:Q8NET5",
  "gene_symbol": "NFAM1",
  "term_label": "calcineurin-NFAT signaling cascade",
  "gene_name": "NFAT activation molecule 1"
}